{
  "term_id": "GO:0008139",
  "term_label": "nuclear localization sequence binding",
  "gene": "UniProtKB:A6NF01",
  "gene_symbol": "POM121B",
  "gene_name": "Putative nuclear envelope pore membrane protein POM 121B"
}